{
  "term_id": "GO:0001708",
  "term_label": "cell fate specification",
  "gene_symbol": "TBX6",
  "gene_name": "T-box transcription factor TBX6",
  "gene": "UniProtKB:O95947"
}